{
  "gene_name": "Biogenesis of lysosome-related organelles complex 1 subunit 4",
  "gene_symbol": "BLOC1S4",
  "gene": "UniProtKB:Q9NUP1",
  "term_id": "GO:0031083",
  "term_label": "BLOC-1 complex"
}